{
  "gene_symbol": "CAPN8",
  "term_label": "calcium-dependent cysteine-type endopeptidase activity",
  "gene": "UniProtKB:A6NHC0",
  "term_id": "GO:0004198",
  "gene_name": "Calpain-8"
}